{
  "gene_name": "Zona pellucida-like domain-containing protein 1",
  "gene": "UniProtKB:Q8TCW7",
  "term_label": "extracellular space",
  "gene_symbol": "ZPLD1",
  "term_id": "GO:0005615"
}